{
  "term_label": "G protein-coupled purinergic nucleotide receptor activity",
  "gene_name": "G-protein coupled receptor 87",
  "gene_symbol": "GPR87",
  "gene": "UniProtKB:Q9BY21",
  "term_id": "GO:0045028"
}